{
  "gene_symbol": "UGT1A8",
  "gene_name": "UDP-glucuronosyltransferase 1A8",
  "term_id": "GO:0008194",
  "gene": "UniProtKB:Q9HAW9",
  "term_label": "UDP-glycosyltransferase activity"
}